{
  "term_label": "Unknown cellular component",
  "gene_name": "Keratin-associated protein 10-10",
  "gene_symbol": "KRTAP10-10",
  "gene": "UniProtKB:P60014",
  "term_id": "UNKNOWN:0003"
}